{
  "term_label": "DNA-binding transcription repressor activity, RNA polymerase II-specific",
  "gene": "UniProtKB:Q86T24",
  "term_id": "GO:0001227",
  "gene_name": "Transcriptional regulator Kaiso",
  "gene_symbol": "ZBTB33"
}